gamma-tubulin complex binding [GO:0140496] (molecular function) Definition: Binding to a gamma-tubulin complex. References: PMID:30174135 Relationships: is a type of protein-containing complex binding [GO:0044877]